{
  "gene_symbol": "PON3",
  "term_id": "GO:0004064",
  "gene": "UniProtKB:Q15166",
  "gene_name": "Serum paraoxonase_lactonase 3",
  "term_label": "arylesterase activity"
}